{
  "gene_name": "Glycogen phosphorylase, muscle form",
  "term_id": "GO:0005980",
  "gene_symbol": "PYGM",
  "gene": "UniProtKB:P11217",
  "term_label": "glycogen catabolic process"
}